{
  "term_label": "Unknown molecular function",
  "gene_symbol": "PMPCA",
  "gene_name": "Mitochondrial-processing peptidase subunit alpha",
  "term_id": "UNKNOWN:0001",
  "gene": "UniProtKB:Q10713"
}